{
  "term_id": "GO:0046381",
  "gene": "UniProtKB:Q9Y471",
  "term_label": "CMP-N-acetylneuraminate metabolic process",
  "gene_name": "Inactive cytidine monophosphate-N-acetylneuraminic acid hydroxylase",
  "gene_symbol": "CMAHP"
}